{
  "term_id": "GO:0003723",
  "term_label": "RNA binding",
  "gene_name": "RNA-binding protein 45",
  "gene_symbol": "RBM45",
  "gene": "UniProtKB:Q8IUH3"
}